{
  "gene_symbol": "NOX4",
  "term_label": "plasma membrane",
  "term_id": "GO:0005886",
  "gene": "UniProtKB:Q9NPH5",
  "gene_name": "NADPH oxidase 4"
}